{
  "gene": "UniProtKB:P07864",
  "term_id": "GO:0005739",
  "gene_symbol": "LDHC",
  "term_label": "mitochondrion",
  "gene_name": "L-lactate dehydrogenase C chain"
}